{
  "term_label": "axon",
  "gene_name": "Potassium voltage-gated channel subfamily A member 4",
  "gene": "UniProtKB:P22459",
  "term_id": "GO:0030424",
  "gene_symbol": "KCNA4"
}